{
  "term_id": "UNKNOWN:0001",
  "gene_symbol": "HILPDA",
  "gene_name": "Hypoxia-inducible lipid droplet-associated protein",
  "term_label": "Unknown molecular function",
  "gene": "UniProtKB:Q9Y5L2"
}